{
  "gene": "UniProtKB:Q05707",
  "term_id": "UNKNOWN:0001",
  "term_label": "Unknown molecular function",
  "gene_name": "Collagen alpha-1(XIV) chain",
  "gene_symbol": "COL14A1"
}